{
  "term_id": "UNKNOWN:0002",
  "gene": "UniProtKB:A6NEH8",
  "gene_name": "Putative uncharacterized protein encoded by ZNF503-AS2",
  "term_label": "Unknown biological process",
  "gene_symbol": "ZNF503-AS2"
}